{
  "term_id": "GO:0004984",
  "gene_symbol": "OR5B12",
  "gene": "UniProtKB:Q96R08",
  "term_label": "olfactory receptor activity",
  "gene_name": "Olfactory receptor 5B12"
}